axon ensheathment [GO:0008366] (biological process) Sources: GOC:jl, ISBN:0878932437 Also known as: cellular axon ensheathment, cellular nerve ensheathment, nerve ensheathment Definition: Any process in which the axon of a neuron is insulated, and that insulation maintained, thereby preventing dispersion of the electrical signal. Subtypes: non-myelinated axon ensheathment [GO:0032285], axon ensheathment in central nervous system [GO:0032291], GO:0032292, GO:0042552, glial cell projection elongation involved in axon ensheathment [GO:0106092] Relationships: is a type of GO:0007272